{
  "gene_symbol": "THY1",
  "term_id": "GO:0045121",
  "gene": "UniProtKB:P04216",
  "term_label": "membrane raft",
  "gene_name": "Thy-1 membrane glycoprotein"
}